{
  "gene_symbol": "H1-1",
  "term_label": "nucleosomal DNA binding",
  "gene": "UniProtKB:Q02539",
  "term_id": "GO:0031492",
  "gene_name": "Histone H1.1"
}